{
  "term_id": "GO:0009897",
  "gene_name": "Erythropoietin receptor",
  "term_label": "external side of plasma membrane",
  "gene": "UniProtKB:P19235",
  "gene_symbol": "EPOR"
}